{
  "gene_symbol": "SOAT2",
  "gene": "UniProtKB:O75908",
  "term_label": "cholesterol metabolic process",
  "gene_name": "Sterol O-acyltransferase 2",
  "term_id": "GO:0008203"
}